{
  "gene": "UniProtKB:Q96I45",
  "gene_symbol": "TMEM141",
  "term_id": "UNKNOWN:0003",
  "term_label": "Unknown cellular component",
  "gene_name": "Transmembrane protein 141"
}